{
  "term_label": "ubiquitin protein ligase activity",
  "gene": "UniProtKB:Q9BVG3",
  "gene_symbol": "TRIM62",
  "term_id": "GO:0061630",
  "gene_name": "E3 ubiquitin-protein ligase TRIM62"
}